{
  "term_id": "GO:0110031",
  "gene_name": "Serine_threonine-protein kinase 35",
  "gene_symbol": "STK35",
  "gene": "UniProtKB:Q8TDR2",
  "term_label": "negative regulation of G2/MI transition of meiotic cell cycle"
}